{
  "gene": "UniProtKB:Q96JH7",
  "term_label": "cysteine-type deubiquitinase activity",
  "gene_symbol": "VCPIP1",
  "gene_name": "Deubiquitinating protein VCPIP1",
  "term_id": "GO:0004843"
}